scavenger receptor activity [GO:0005044] (molecular function) Also known as: macrophage receptor activity Note: Note that many gene products that are called scavenger receptors have a broad range of potential ligands and also can be annotated to 'pattern recognition receptor activity ; GO:0038187' or its child terms, or to 'lipoprotein receptor activity ; GO:0030228' or its child terms. For receptors that transduce a signal rather than endocytose their ligand, consider instead the terms 'signaling receptor activity ; GO:0038023' and its children. Relationships: is a type of cargo receptor activity [GO:0038024] Definition: Combining with any modified low-density lipoprotein (LDL) or other polyanionic ligand and delivering the ligand into the cell via endocytosis. Ligands include acetylated and oxidized LDL, Gram-positive and Gram-negative bacteria, apoptotic cells, amyloid-beta fibrils, and advanced glycation end products (AGEs). References: PMID:11790542, PMID:12379907, PMID:12621157, PMID:20981357 Sources: GOC:bf